{
  "gene": "UniProtKB:Q9H159",
  "gene_name": "Cadherin-19",
  "term_label": "catenin complex",
  "gene_symbol": "CDH19",
  "term_id": "GO:0016342"
}